sarsapogenin 3-beta-glucosyltransferase activity [GO:0047249] (molecular function) Also known as: UDP-glucose:(25S)-5beta-spirostan-3beta-ol 3-O-beta-D-glucosyltransferase activity, UDPglucose:(25S)-5beta-spirostan-3beta-ol 3-O-beta-D-glucosyltransferase activity, sarsapogenin 3beta-glucosyltransferase activity, uridine diphosphoglucose-sarsapogenin glucosyltransferase activity Definition: Catalysis of the reaction: (25S)-5beta-spirostan-3beta-ol + UDP-D-glucose = (25S)-5beta-spirostan-3beta-yl beta-D-glucoside + H+ + UDP. Relationships: is a type of UDP-glucosyltransferase activity [GO:0035251] Sources: EC:2.4.1.193, RHEA:14461